{
  "term_id": "GO:0015279",
  "gene_symbol": "TRPC6",
  "gene_name": "Short transient receptor potential channel 6",
  "gene": "UniProtKB:Q9Y210",
  "term_label": "store-operated calcium channel activity"
}